{
  "gene": "UniProtKB:O60469",
  "gene_name": "Cell adhesion molecule DSCAM",
  "term_label": "positive regulation of axon extension involved in axon guidance",
  "term_id": "GO:0048842",
  "gene_symbol": "DSCAM"
}